{
  "term_label": "endopeptidase activator activity",
  "term_id": "GO:0061133",
  "gene_symbol": "ADRM1",
  "gene_name": "Proteasomal ubiquitin receptor ADRM1",
  "gene": "UniProtKB:Q16186"
}